fatty acid synthase activity [GO:0004312] (molecular function) Definition: Catalysis of the reaction: acetyl-CoA + n malonyl-CoA + 2n NADPH + 2n H+ = long-chain fatty acid + n+1 CoA + n CO2 + 2n NADP+. Relationships: is a type of acyltransferase activity, transferring groups other than amino-acyl groups [GO:0016747] Also known as: fatty-acid synthase activity, acyl-CoA:malonyl-CoA C-acyltransferase (decarboxylating, oxoacyl- and enoyl-reducing and thioester-hydrolysing) Sources: EC:2.3.1.85